{
  "term_label": "Unknown biological process",
  "gene_name": "Putative E3 ubiquitin-protein ligase UNKL",
  "term_id": "UNKNOWN:0002",
  "gene_symbol": "UNKL",
  "gene": "UniProtKB:Q9H9P5"
}